phthalate 3,4-cis-dihydrodiol dehydrogenase activity [GO:0034912] (molecular function) Sources: UM-BBD_reactionID:r1445 Definition: Catalysis of the reaction: phthalate 3,4-cis-dihydrodiol + NAD+ = 3,4-dihydroxyphthalate + NADH + H+. Relationships: is a type of oxidoreductase activity, acting on the CH-CH group of donors, NAD or NADP as acceptor [GO:0016628]